{
  "gene_name": "Ubiquitin carboxyl-terminal hydrolase 17-like protein 10",
  "term_label": "cytosol",
  "term_id": "GO:0005829",
  "gene_symbol": "USP17L10",
  "gene": "UniProtKB:C9JJH3"
}